reproductive process in single-celled organism [GO:0022413] (biological process) Sources: GOC:isa_complete Definition: A process, occurring at the cellular level, that is involved in the reproductive function of a single-celled organism. Subtypes: GO:0000755, cell budding [GO:0007114], GO:0007533, ascospore formation [GO:0030437], actinomycete-type spore formation [GO:0034304], GO:0043093, mating-type locus imprinting [GO:0071515], sexual macrocyst formation [GO:0140084] Relationships: is a type of reproductive process [GO:0022414]